{
  "gene_name": "Protein maelstrom homolog",
  "term_label": "nucleus",
  "gene_symbol": "MAEL",
  "gene": "UniProtKB:Q96JY0",
  "term_id": "GO:0005634"
}